{
  "term_id": "GO:0005886",
  "gene": "UniProtKB:Q8NH56",
  "term_label": "plasma membrane",
  "gene_symbol": "OR52N5",
  "gene_name": "Olfactory receptor 52N5"
}